{
  "gene": "UniProtKB:Q9Y6V0",
  "term_label": "structural constituent of presynaptic active zone",
  "term_id": "GO:0098882",
  "gene_name": "Protein piccolo",
  "gene_symbol": "PCLO"
}